{
  "term_id": "GO:0003697",
  "term_label": "single-stranded DNA binding",
  "gene_name": "Single-stranded DNA-binding protein, mitochondrial",
  "gene": "UniProtKB:Q04837",
  "gene_symbol": "SSBP1"
}